{
  "term_id": "GO:0001514",
  "gene_name": "tRNA selenocysteine 1-associated protein 1",
  "gene_symbol": "TRNAU1AP",
  "gene": "UniProtKB:Q9NX07",
  "term_label": "selenocysteine incorporation"
}